{
  "gene_name": "Cytochrome P450 11B2, mitochondrial",
  "gene_symbol": "CYP11B2",
  "term_id": "GO:0004507",
  "term_label": "steroid 11-beta-monooxygenase activity",
  "gene": "UniProtKB:P19099"
}